{
  "term_id": "UNKNOWN:0002",
  "gene_symbol": "YIPF6",
  "gene_name": "Protein YIPF6",
  "term_label": "Unknown biological process",
  "gene": "UniProtKB:Q96EC8"
}